regulation of response to external stimulus [GO:0032101] (biological process) Sources: GOC:mah Note: Note that this term is in the subset of terms that should not be used for direct gene product annotation. Instead, select a child term or, if no appropriate child term exists, please request a new term. Direct annotations to this term may be amended during annotation QC. Subtypes: regulation of antimicrobial humoral response [GO:0002759], regulation of systemic acquired resistance [GO:0010112], regulation of opsin-mediated signaling pathway [GO:0022400], regulation of blood coagulation [GO:0030193], regulation of lipopolysaccharide-mediated signaling pathway [GO:0031664], GO:0032102, positive regulation of response to external stimulus [GO:0032103], regulation of skeletal muscle tissue regeneration [GO:0043416], GO:0045088, GO:0048679, regulation of defense response to virus [GO:0050688], regulation of inflammatory response [GO:0050727], regulation of chemotaxis [GO:0050920], regulation of neutrophil mediated killing of symbiont cell [GO:0070949], regulation of defense response to fungus [GO:1900150], regulation of defense response to bacterium [GO:1900424], GO:1902288, GO:1904365, regulation of xenophagy [GO:1904415], GO:1905787, regulation of mechanosensory behavior [GO:1905790], GO:2000068 Relationships: is a type of regulation of response to stimulus [GO:0048583]; regulates response to external stimulus [GO:0009605] Definition: Any process that modulates the frequency, rate or extent of a response to an external stimulus.